{
  "gene_symbol": "WDR24",
  "gene_name": "GATOR complex protein WDR24",
  "term_id": "GO:1904263",
  "gene": "UniProtKB:Q96S15",
  "term_label": "positive regulation of TORC1 signaling"
}